{
  "gene_symbol": "IZUMO4",
  "term_id": "UNKNOWN:0002",
  "gene_name": "Izumo sperm-egg fusion protein 4",
  "gene": "UniProtKB:Q1ZYL8",
  "term_label": "Unknown biological process"
}